{
  "term_id": "GO:0005739",
  "gene_name": "tRNA N6-adenosine threonylcarbamoyltransferase, mitochondrial",
  "gene_symbol": "OSGEPL1",
  "term_label": "mitochondrion",
  "gene": "UniProtKB:Q9H4B0"
}